{
  "gene_name": "F-box only protein 3",
  "term_id": "UNKNOWN:0002",
  "gene": "UniProtKB:Q9UK99",
  "term_label": "Unknown biological process",
  "gene_symbol": "FBXO3"
}